{
  "gene": "UniProtKB:O60662",
  "term_id": "GO:0045661",
  "gene_symbol": "KLHL41",
  "term_label": "regulation of myoblast differentiation",
  "gene_name": "Kelch-like protein 41"
}